{
  "term_id": "GO:0005634",
  "gene_name": "DNA_RNA-binding protein KIN17",
  "gene_symbol": "KIN",
  "term_label": "nucleus",
  "gene": "UniProtKB:O60870"
}